Toll-like receptor 4 binding [GO:0035662] (molecular function) Definition: Binding to a Toll-like 4 protein, a pattern recognition receptor that binds bacterial lipopolysaccharide (LPS) to initiate an innate immune response. References: PMID:18304834 Sources: GOC:BHF Also known as: TLR4 binding Relationships: is a type of Toll-like receptor binding [GO:0035325]